{
  "gene_symbol": "HSPA1B",
  "gene_name": "Heat shock 70 kDa protein 1B",
  "term_id": "GO:0005829",
  "gene": "UniProtKB:P0DMV9",
  "term_label": "cytosol"
}